{
  "term_label": "RNA binding",
  "gene": "UniProtKB:O75683",
  "term_id": "GO:0003723",
  "gene_name": "Surfeit locus protein 6",
  "gene_symbol": "SURF6"
}